maltodextrin transmembrane transporter activity [GO:0042958] (molecular function) Definition: Enables the transfer of maltodextrin, any polysaccharide of glucose residues in beta-(1,4) linkage, from one side of a membrane to the other. References: PMID:15034926 Sources: GOC:jl Relationships: is a type of dextrin transmembrane transporter activity [GO:0042957]; is part of maltodextrin transmembrane transport [GO:0042956]